{
  "term_label": "microtubule-based movement",
  "gene_name": "Dynein light chain Tctex-type 1",
  "gene_symbol": "DYNLT1",
  "gene": "UniProtKB:P63172",
  "term_id": "GO:0007018"
}